zeaxanthin biosynthetic process [GO:1901827] (biological process) Definition: The chemical reactions and pathways resulting in the formation of zeaxanthin. Relationships: is a type of xanthophyll biosynthetic process [GO:0016123] Sources: GOC:TermGenie, GOC:yaf, MetaCyc:PWY-5944, UniPathway:UPA00843 Also known as: zeaxanthin anabolism, zeaxanthin biosynthesis, zeaxanthin formation, zeaxanthin synthesis